inositol 2-dehydrogenase (NAD+) activity [GO:0050112] (molecular function) Relationships: is_a alcohol dehydrogenase (NAD+) activity [GO:0004022] Definition: Catalysis of the reaction: myo-inositol + NAD+ = 2,4,6/3,5-pentahydroxycyclohexanone + H+ + NADH. Sources: EC:1.1.1.18, RHEA:16949 Also known as: inositol 2-dehydrogenase activity, inositol:NAD 2-dehydrogenase activity, myo-inositol 2-dehydrogenase activity